{
  "gene_name": "Apolipoprotein B receptor",
  "term_id": "GO:0016020",
  "gene": "UniProtKB:Q0VD83",
  "term_label": "membrane",
  "gene_symbol": "APOBR"
}